{
  "term_label": "catalytic step 2 spliceosome",
  "term_id": "GO:0071013",
  "gene_symbol": "LSM3",
  "gene": "UniProtKB:P62310",
  "gene_name": "U6 snRNA-associated Sm-like protein LSm3"
}